subsynaptic reticulum organization [GO:1990255] (biological process) References: PMID:21041451 Relationships: is a type of GO:0006996 Definition: A process that is carried out at the cellular level which results in the assembly, arrangement of constituent parts, or disassembly of a subsynaptic reticulum. A subsynaptic reticulum is an elaborate tubulolamellar membrane system that underlies the postsynaptic cell membrane.